{
  "gene": "UniProtKB:Q9H7L2",
  "term_label": "plasma membrane",
  "term_id": "GO:0005886",
  "gene_symbol": "KIR3DX1",
  "gene_name": "Putative killer cell immunoglobulin-like receptor-like protein KIR3DX1"
}